{
  "term_label": "cytoplasm",
  "gene_symbol": "DNAAF11",
  "gene_name": "Dynein axonemal assembly factor 11",
  "gene": "UniProtKB:Q86X45",
  "term_id": "GO:0005737"
}